positive regulation of egg-laying behavior [GO:1901046] (biological process) Definition: Any process that activates or increases the frequency, rate or extent of oviposition. Relationships: is a type of regulation of egg-laying behavior [GO:0046662]; is a type of positive regulation of behavior [GO:0048520]; is a type of positive regulation of reproductive process [GO:2000243]; positively regulates egg-laying behavior [GO:0018991] Also known as: activation of egg laying, activation of egg-laying, positive regulation of egg laying, positive regulation of egg-laying, up regulation of egg laying, up regulation of egg-laying, up-regulation of egg laying, up-regulation of egg-laying, upregulation of egg laying, upregulation of egg-laying, positive regulation of oviposition, up regulation of oviposition, up-regulation of oviposition, upregulation of oviposition, activation of oviposition Sources: GOC:TermGenie, GOC:kmv